{
  "gene_name": "Disintegrin and metalloproteinase domain-containing protein 19",
  "gene_symbol": "ADAM19",
  "term_id": "UNKNOWN:0003",
  "term_label": "Unknown cellular component",
  "gene": "UniProtKB:Q9H013"
}